(-)-lariciresinol biosynthetic process [GO:1902129] (biological process) Also known as: (-)-lariciresinol anabolism, (-)-lariciresinol biosynthesis, (-)-lariciresinol formation, (-)-lariciresinol synthesis Relationships: is a type of lignan biosynthetic process [GO:0009807]; is a type of GO:0046189 References: PMID:15949826, PMID:9872995 Sources: GOC:TermGenie Definition: The chemical reactions and pathways resulting in the formation of (-)-lariciresinol.